{
  "term_id": "GO:0005739",
  "gene": "UniProtKB:Q4VC31",
  "gene_name": "Protein MIX23",
  "gene_symbol": "MIX23",
  "term_label": "mitochondrion"
}